response to nitrosative stress [GO:0051409] (biological process) Subtypes: GO:0071500 References: PMID:15925705 Definition: Any process that results in a change in state or activity of a cell or an organism (in terms of movement, secretion, enzyme production, gene expression, etc.) as a result of a nitrosative stress stimulus. Nitrosative stress is a state often resulting from exposure to high levels of nitric oxide (NO) or the highly reactive oxidant peroxynitrite, which is produced following interaction of NO with superoxide anions. Relationships: is a type of GO:0006950